{
  "gene_symbol": "LHFPL5",
  "term_label": "plasma membrane",
  "gene": "UniProtKB:Q8TAF8",
  "gene_name": "LHFPL tetraspan subfamily member 5 protein",
  "term_id": "GO:0005886"
}